mitochondrial respiratory chain complex IV assembly [GO:0033617] (biological process) Definition: The aggregation, arrangement and bonding together of a set of components to form respiratory chain complex IV (also known as cytochrome c oxidase) in the mitochondrial inner membrane. Sources: GOC:mah Also known as: mitochondrial cytochrome c oxidase biogenesis, mitochondrial cytochrome c oxidase assembly, mitochondrial cytochrome c oxidase complex assembly Relationships: is_a GO:0008535; is a type of mitochondrial respiratory chain complex assembly [GO:0033108]